{
  "gene_name": "DNA-binding protein inhibitor ID-3",
  "term_label": "negative regulation of transcription by RNA polymerase II",
  "gene_symbol": "ID3",
  "term_id": "GO:0000122",
  "gene": "UniProtKB:Q02535"
}